{
  "gene_name": "Clusterin-like protein 1",
  "term_label": "misfolded protein binding",
  "gene_symbol": "CLUL1",
  "term_id": "GO:0051787",
  "gene": "UniProtKB:Q15846"
}